negative regulation of neuron migration [GO:2001223] (biological process) Also known as: negative regulation of neuron chemotaxis, negative regulation of neuronal migration, negative regulation of neuron guidance Subtypes: negative regulation of motor neuron migration [GO:1905484] Relationships: is a type of GO:0030336; is a type of regulation of neuron migration [GO:2001222]; negatively regulates neuron migration [GO:0001764] Sources: GOC:obol Definition: Any process that stops, prevents or reduces the frequency, rate or extent of neuron migration.